{
  "gene": "UniProtKB:Q5VTH9",
  "gene_symbol": "DNAI4",
  "term_id": "GO:0045503",
  "term_label": "dynein light chain binding",
  "gene_name": "Dynein axonemal intermediate chain 4"
}